{
  "gene": "UniProtKB:Q9UKB5",
  "gene_name": "Adherens junction-associated protein 1",
  "term_label": "adherens junction",
  "gene_symbol": "AJAP1",
  "term_id": "GO:0005912"
}